transcription factor TFIID complex [GO:0005669] (cellular component) Relationships: is_a RNA polymerase II transcription regulator complex [GO:0090575]; is part of GO:0016591 Subtypes: TAF4B-containing transcription factor TFIID complex [GO:0070556] Sources: GOC:krc, GOC:mah, ISBN:0471953393, ISBN:0879695501 Definition: A complex composed of TATA binding protein (TBP) and TBP associated factors (TAFs); the total mass is typically about 800 kDa. Most of the TAFs are conserved across species. In TATA-containing promoters for RNA polymerase II (Pol II), TFIID is believed to recognize at least two distinct elements, the TATA element and a downstream promoter element. TFIID is also involved in recognition of TATA-less Pol II promoters. Binding of TFIID to DNA is necessary but not sufficient for transcription initiation from most RNA polymerase II promoters.